{
  "term_label": "regulation of systemic arterial blood pressure",
  "gene_name": "Pro-adrenomedullin",
  "term_id": "GO:0003073",
  "gene": "UniProtKB:P35318",
  "gene_symbol": "ADM"
}